arogenate dehydrogenase [NAD(P)+] activity [GO:0033731] (molecular function) Relationships: is a type of oxidoreductase activity, acting on the CH-CH group of donors, NAD or NADP as acceptor [GO:0016628] Definition: Catalysis of the reaction: L-arogenate + NAD(P)+ = L-tyrosine + NAD(P)H + CO2. Sources: EC:1.3.1.79 Subtypes: arogenate dehydrogenase (NADP+) activity [GO:0033730] Also known as: arogenic dehydrogenase activity, pretyrosine dehydrogenase activity, L-arogenate:NAD(P)+ oxidoreductase (decarboxylating) activity